sulfide oxidation, using sulfur dioxygenase [GO:0070223] (biological process) Definition: A sulfide oxidation process that proceeds via the reaction catalyzed by sulfur dioxygenase. Also known as: sulphide oxidation, using sulfur dioxygenase Relationships: is a type of GO:0019418 Sources: MetaCyc:PWY-5285